{
  "gene_symbol": "HES7",
  "gene": "UniProtKB:Q9BYE0",
  "gene_name": "Transcription factor HES-7",
  "term_id": "GO:0009952",
  "term_label": "anterior/posterior pattern specification"
}